cysteine-type aminopeptidase activity [GO:0070005] (MF) Sources: GOC:mah, https://www.ebi.ac.uk/merops/about/glossary.shtml#AMINOPEPTIDASE, https://www.ebi.ac.uk/merops/about/glossary.shtml#CATTYPE Definition: Catalysis of the hydrolysis of a single N-terminal amino acid residue from a polypeptide chain by a mechanism in which the sulfhydryl group of a cysteine residue at the active center acts as a nucleophile. Relationships: is a type of aminopeptidase activity [GO:0004177]; is a type of cysteine-type exopeptidase activity [GO:0070004]